bud dilation involved in lung branching [GO:0060503] (biological process) Definition: The process in which a bud in the lung increases radially. Also known as: bud expansion Relationships: is a type of axis elongation [GO:0003401]; is part of epithelial tube branching involved in lung morphogenesis [GO:0060441] Sources: GOC:dph